{
  "gene": "UniProtKB:Q15392",
  "gene_symbol": "DHCR24",
  "term_label": "steroid metabolic process",
  "gene_name": "Delta(24)-sterol reductase",
  "term_id": "GO:0008202"
}